{
  "gene_symbol": "MEAK7",
  "term_label": "TOR signaling",
  "term_id": "GO:0031929",
  "gene_name": "MTOR-associated protein MEAK7",
  "gene": "UniProtKB:Q6P9B6"
}